{
  "term_id": "GO:0031463",
  "gene": "UniProtKB:Q2TBA0",
  "gene_name": "Kelch-like protein 40",
  "gene_symbol": "KLHL40",
  "term_label": "Cul3-RING ubiquitin ligase complex"
}